platelet-derived growth factor receptor binding [GO:0005161] (molecular function) Sources: GOC:ai Also known as: PDGF receptor binding, PDGFR binding, PDGF, platelet-derived growth factor, platelet-derived growth factor receptor ligand Definition: Binding to a platelet-derived growth factor receptor. Relationships: is a type of GO:0070851